{
  "gene_name": "WD repeat-containing protein 18",
  "gene": "UniProtKB:Q9BV38",
  "term_label": "rixosome complex",
  "term_id": "GO:0120330",
  "gene_symbol": "WDR18"
}